{
  "gene_symbol": "TLX1",
  "term_id": "GO:0005634",
  "gene_name": "T-cell leukemia homeobox protein 1",
  "gene": "UniProtKB:P31314",
  "term_label": "nucleus"
}